saccharopine dehydrogenase (NADP+, L-glutamate-forming) activity [GO:0004755] (molecular function) Definition: Catalysis of the reaction: L-saccharopine + H2O + NADP+ = L-allysine + L-glutamate + H+ + NADPH. Sources: EC:1.5.1.10, RHEA:10020 Relationships: is a type of saccharopine dehydrogenase activity [GO:0004753] Also known as: 6-N-(L-1,3-dicarboxypropyl)-L-lysine:NADP+ oxidoreductase (L-glutamate-forming), N6-(L-1,3-dicarboxypropyl)-L-lysine:NADP+ oxidoreductase (L-glutamate-forming), aminoadipate semialdehyde-glutamate reductase activity, aminoadipic semialdehyde-glutamate reductase activity, aminoadipic semialdehyde-glutamic reductase activity, epsilon-N-(L-glutaryl-2)-L-lysine:NAD+(P) oxidoreductase (L-2-aminoadipate-semialdehyde forming), saccharopine (nicotinamide adenine dinucleotide phosphate, glutamate-forming) dehydrogenase activity, saccharopine reductase activity